{
  "term_id": "GO:0030159",
  "gene": "UniProtKB:Q13322",
  "gene_name": "Growth factor receptor-bound protein 10",
  "term_label": "signaling receptor complex adaptor activity",
  "gene_symbol": "GRB10"
}